{
  "gene": "UniProtKB:Q05BV3",
  "gene_name": "Echinoderm microtubule-associated protein-like 5",
  "term_label": "microtubule binding",
  "term_id": "GO:0008017",
  "gene_symbol": "EML5"
}